{
  "term_label": "cell-cell signaling",
  "gene": "UniProtKB:O95377",
  "gene_symbol": "GJB5",
  "term_id": "GO:0007267",
  "gene_name": "Gap junction beta-5 protein"
}